{
  "term_id": "GO:0005385",
  "gene": "UniProtKB:Q504Y0",
  "gene_symbol": "SLC39A12",
  "term_label": "zinc ion transmembrane transporter activity",
  "gene_name": "Zinc transporter ZIP12"
}